regulation of embryonic camera-type eye development [GO:1902863] (biological process) Definition: Any process that modulates the frequency, rate or extent of embryonic camera-type eye development. Also known as: regulation of embryonic eye development Subtypes: negative regulation of embryonic camera-type eye development [GO:1902864], positive regulation of embryonic camera-type eye development [GO:1902865] References: PMID:16872597 Sources: GOC:TermGenie, GOC:mr, GO_REF:0000058 Relationships: is a type of GO:0050793; regulates embryonic camera-type eye development [GO:0031076]